{
  "term_label": "Unknown molecular function",
  "gene_name": "Testis-expressed protein 30",
  "gene_symbol": "TEX30",
  "gene": "UniProtKB:Q5JUR7",
  "term_id": "UNKNOWN:0001"
}